{
  "gene_name": "LYR motif-containing protein 1",
  "gene": "UniProtKB:O43325",
  "gene_symbol": "LYRM1",
  "term_label": "Unknown molecular function",
  "term_id": "UNKNOWN:0001"
}